{
  "gene_name": "Nucleolar protein 4",
  "gene_symbol": "NOL4",
  "term_id": "UNKNOWN:0003",
  "term_label": "Unknown cellular component",
  "gene": "UniProtKB:O94818"
}